response to Aroclor 1254 [GO:1904010] (biological process) Definition: Any process that results in a change in state or activity of a cell or an organism (in terms of movement, secretion, enzyme production, gene expression, etc.) as a result of an Aroclor 1254 stimulus. Relationships: is a type of response to chemical [GO:0042221] References: PMID:18602130 Sources: GOC:TermGenie, GO_REF:0000071 Subtypes: cellular response to Aroclor 1254 [GO:1904011]